skeletal muscle satellite cell migration [GO:1902766] (biological process) References: PMID:17996437, PMID:19609936 Sources: GOC:TermGenie, GOC:mr, GO_REF:0000091 Relationships: is a type of cell migration [GO:0016477] Definition: The orderly movement of a skeletal muscle satellite cell from one site to another. Migration of these cells is a key step in the process of growth and repair of skeletal muscle cells.